{
  "term_label": "DNA-binding transcription factor activity, RNA polymerase II-specific",
  "gene": "UniProtKB:P10071",
  "term_id": "GO:0000981",
  "gene_symbol": "GLI3",
  "gene_name": "Transcriptional activator GLI3"
}